{
  "gene_name": "Protein phosphatase 1L",
  "gene_symbol": "PPM1L",
  "term_label": "protein serine/threonine phosphatase activity",
  "gene": "UniProtKB:Q5SGD2",
  "term_id": "GO:0004722"
}